oxidoreductase activity, acting on the CH-NH group of donors, quinone or similar compound as acceptor [GO:0016649] (MF) Definition: Catalysis of an oxidation-reduction (redox) reaction in which a CH-NH group acts as a hydrogen or electron donor and reduces quinone or similar compound. Sources: GOC:jl Subtypes: electron-transferring-flavoprotein dehydrogenase activity [GO:0004174], proline dehydrogenase activity [GO:0004657] Relationships: is a type of oxidoreductase activity, acting on the CH-NH group of donors [GO:0016645]